{
  "term_label": "axon",
  "gene_name": "Ras-related protein Rab-5A",
  "term_id": "GO:0030424",
  "gene_symbol": "RAB5A",
  "gene": "UniProtKB:P20339"
}